positive regulation of interleukin-6 production [GO:0032755] (biological process) Sources: GOC:mah Definition: Any process that activates or increases the frequency, rate, or extent of interleukin-6 production. Also known as: positive regulation of IL-6 production, up regulation of interleukin-6 production, up-regulation of interleukin-6 production, upregulation of interleukin-6 production, activation of interleukin-6 production, positive regulation of interleukin-6 biosynthetic process, positive regulation of interleukin-6 secretion, stimulation of interleukin-6 production Relationships: is a type of GO:0001819; is a type of regulation of interleukin-6 production [GO:0032675]; positively regulates GO:0032635